{
  "gene_symbol": "SLC25A22",
  "term_id": "GO:0005313",
  "term_label": "L-glutamate transmembrane transporter activity",
  "gene": "UniProtKB:Q9H936",
  "gene_name": "Mitochondrial glutamate carrier 1"
}